positive regulation of secondary growth [GO:2000605] (biological process) Definition: Any process that activates or increases the frequency, rate or extent of secondary growth. Relationships: is a type of positive regulation of growth [GO:0045927]; is a type of GO:2000603; positively regulates secondary growth [GO:0080117] Sources: GOC:obol